mitotic prometaphase [GO:0000236] (biological process) Definition: The cell cycle phase in higher eukaryotes which follows mitotic prophase and during which the nuclear envelope is disrupted and breaks into membrane vesicles, and the spindle microtubules enter the nuclear region. Kinetochores mature on each centromere and attach to some of the spindle microtubules. Kinetochore microtubules begin the process of aligning chromosomes in one plane halfway between the poles. Sources: GOC:mtg_cell_cycle Note: Note that this term should not be used for direct annotation. If you are trying to make an annotation to x phase, it is likely that the correct annotation is 'regulation of x/y phase transition' or to a process which occurs during the reported phase (i.e mitotic DNA replication for mitotic S-phase). To capture the phase when a specific location or process is observed, the phase term can be used in an annotation extension (PMID:24885854) applied to a cellular component term (with the relation exists_during) or a biological process term (with the relation happens_during). Relationships: is a type of GO:0000087